{
  "term_id": "GO:0005886",
  "gene": "UniProtKB:Q92930",
  "gene_name": "Ras-related protein Rab-8B",
  "term_label": "plasma membrane",
  "gene_symbol": "RAB8B"
}